{
  "term_label": "GTP binding",
  "term_id": "GO:0005525",
  "gene_name": "ADP-ribosylation factor 1",
  "gene": "UniProtKB:P84077",
  "gene_symbol": "ARF1"
}